cellular detoxification of nitrogen compound [GO:0070458] (biological process) Definition: Any cellular process that reduces or removes the toxicity of nitrogenous compounds which are dangerous or toxic. This includes the aerobic conversion of toxic compounds to harmless substances. Sources: GOC:mah Also known as: cellular detoxification of nitrogenous compound Relationships: is a type of GO:0051410; is a type of GO:1990748; is part of cellular response to stress [GO:0033554]